{
  "term_id": "GO:0006357",
  "term_label": "regulation of transcription by RNA polymerase II",
  "gene": "UniProtKB:A0A1W2PPM1",
  "gene_name": "Cytoplasmic polyadenylated homeobox-like protein",
  "gene_symbol": "CPHXL"
}